{
  "gene": "UniProtKB:Q9BXJ5",
  "gene_name": "Complement C1q tumor necrosis factor-related protein 2",
  "term_id": "UNKNOWN:0002",
  "gene_symbol": "C1QTNF2",
  "term_label": "Unknown biological process"
}